{
  "gene": "UniProtKB:Q86SQ4",
  "term_id": "GO:0043236",
  "gene_symbol": "ADGRG6",
  "term_label": "laminin binding",
  "gene_name": "Adhesion G-protein coupled receptor G6"
}